homing of group II introns [GO:0006315] (biological process) References: PMID:10487208 Sources: GOC:mcc, ISBN:0716743663 Relationships: is a type of intron homing [GO:0006314] Definition: Lateral transfer of a group II intron to a homologous allele that lacks the intron, mediated by a site-specific endonuclease encoded within the mobile intron; group II introns are self-splicing introns with a conserved secondary structure.